N-methylnicotinate transport [GO:2001143] (biological process) Sources: GOC:obol Definition: The directed movement of a N-methylnicotinateacetate into, out of or within a cell, or between cells, by means of some agent such as a transporter or pore. Relationships: is_a GO:0015695; is a type of quaternary ammonium group transport [GO:0015697]